{
  "gene_name": "Oxoeicosanoid receptor 1",
  "gene": "UniProtKB:Q8TDS5",
  "gene_symbol": "OXER1",
  "term_id": "GO:0007186",
  "term_label": "G protein-coupled receptor signaling pathway"
}